{
  "gene_name": "Butyrophilin subfamily 3 member A1",
  "term_label": "external side of plasma membrane",
  "term_id": "GO:0009897",
  "gene": "UniProtKB:O00481",
  "gene_symbol": "BTN3A1"
}